negative regulation of activin receptor signaling pathway [GO:0032926] (biological process) Definition: Any process that stops, prevents, or reduces the frequency, rate or extent of the activity of any activin receptor signaling pathway. Subtypes: GO:1900108 Sources: GOC:BHF, GOC:rl Also known as: down regulation of activin receptor signaling pathway, down-regulation of activin receptor signaling pathway, downregulation of activin receptor signaling pathway, negative regulation of activin receptor signalling pathway, inhibition of activin receptor signaling pathway, negative regulation of activin signaling pathway, negative regulation of activin signalling pathway Relationships: is_a regulation of activin receptor signaling pathway [GO:0032925]; is a type of negative regulation of transmembrane receptor protein serine/threonine kinase signaling pathway [GO:0090101]; negatively regulates activin receptor signaling pathway [GO:0032924]